{
  "term_label": "secretory granule",
  "gene": "UniProtKB:Q9UKR0",
  "term_id": "GO:0030141",
  "gene_name": "Kallikrein-12",
  "gene_symbol": "KLK12"
}